auxin transmembrane transporter activity [GO:0080161] (molecular function) Subtypes: GO:0009672, auxin influx transmembrane transporter activity [GO:0010328], auxin efflux transmembrane transporter activity [GO:0010329] Definition: Enables the transfer of auxins from one side of a membrane to the other. Auxins are plant hormones that regulate aspects of plant growth. Relationships: is a type of transmembrane transporter activity [GO:0022857]; is part of auxin transport [GO:0060918] References: PMID:19506555